{
  "gene_name": "Angiomotin-like protein 2",
  "gene": "UniProtKB:Q9Y2J4",
  "term_id": "UNKNOWN:0001",
  "term_label": "Unknown molecular function",
  "gene_symbol": "AMOTL2"
}